{
  "gene": "UniProtKB:Q4VXA5",
  "gene_symbol": "KHDC1",
  "term_label": "RNA binding",
  "gene_name": "KH homology domain-containing protein 1",
  "term_id": "GO:0003723"
}